{
  "gene": "UniProtKB:Q3SXY8",
  "term_label": "non-motile cilium",
  "gene_name": "ADP-ribosylation factor-like protein 13B",
  "term_id": "GO:0097730",
  "gene_symbol": "ARL13B"
}